IDP biosynthetic process [GO:0046708] (BP) Sources: GOC:ai Relationships: is a type of GO:0009152; is a type of purine ribonucleoside diphosphate biosynthetic process [GO:0009180]; is_a IDP metabolic process [GO:0046707] Also known as: IDP anabolism, IDP biosynthesis, IDP formation, IDP synthesis Definition: The chemical reactions and pathways resulting in the formation of IDP, inosine 5'-diphosphate.